{
  "term_label": "nucleus",
  "gene_symbol": "SAP18",
  "gene_name": "Histone deacetylase complex subunit SAP18",
  "gene": "UniProtKB:O00422",
  "term_id": "GO:0005634"
}